{
  "gene": "UniProtKB:O95196",
  "gene_symbol": "CSPG5",
  "term_label": "glial cell projection elongation",
  "gene_name": "Chondroitin sulfate proteoglycan 5",
  "term_id": "GO:0106091"
}